{
  "gene_symbol": "FBXO43",
  "gene": "UniProtKB:Q4G163",
  "gene_name": "F-box only protein 43",
  "term_label": "nucleus",
  "term_id": "GO:0005634"
}